epigenetic programing of female pronucleus [GO:0044726] (biological process) References: PMID:22868271 Sources: GOC:sp Also known as: protection of DNA demethylation of female pronucleus, protection of DNA methylation in female pronucleus, maintenance of DNA methylation at imprinted genes Definition: The global programming of epigenetic modifications in the female pronucleus of the newly fertilized zygote. The maternal genome is protected from global DNA demethylation before the first division of the zygote, and instead undergoes passive, replication-dependent demethylation during early embryogenesis, arising from inhibition of the DNA maintenance methyltransferase Dnmt1. Relationships: is a type of epigenetic programming in the zygotic pronuclei [GO:0044725]